{
  "gene_symbol": "DDX52",
  "term_id": "UNKNOWN:0003",
  "gene": "UniProtKB:Q9Y2R4",
  "term_label": "Unknown cellular component",
  "gene_name": "Probable ATP-dependent RNA helicase DDX52"
}